{
  "gene": "UniProtKB:Q9BZE7",
  "gene_symbol": "C22orf23",
  "term_id": "UNKNOWN:0003",
  "term_label": "Unknown cellular component",
  "gene_name": "UPF0193 protein EVG1"
}